{
  "gene_symbol": "SIX5",
  "term_id": "GO:0000981",
  "gene_name": "Homeobox protein SIX5",
  "gene": "UniProtKB:Q8N196",
  "term_label": "DNA-binding transcription factor activity, RNA polymerase II-specific"
}